sarcosine N-methyltransferase activity [GO:0052730] (molecular function) Sources: RHEA:15453 Relationships: is a type of N-methyltransferase activity [GO:0008170]; is_a S-adenosylmethionine-dependent methyltransferase activity [GO:0008757] Also known as: S-adenosyl-L-methionine:N,N-sarcosine N-methyltransferase activity, SDMT Definition: Catalysis of the reaction: S-adenosyl-L-methionine + sarcosine = S-adenosyl-L-homocysteine + N,N-dimethylglycine.